{
  "gene": "UniProtKB:Q9UBS9",
  "gene_symbol": "SUCO",
  "term_id": "UNKNOWN:0001",
  "gene_name": "SUN domain-containing ossification factor",
  "term_label": "Unknown molecular function"
}